{
  "term_id": "UNKNOWN:0003",
  "gene_symbol": "TSEN34",
  "term_label": "Unknown cellular component",
  "gene_name": "tRNA-splicing endonuclease subunit Sen34",
  "gene": "UniProtKB:Q9BSV6"
}